acetylcholine biosynthetic process [GO:0008292] (biological process) Also known as: acetylcholine anabolism, acetylcholine biosynthesis, acetylcholine formation, acetylcholine synthesis Sources: GOC:jl, ISBN:0192800752 Regulation: regulated by regulation of acetylcholine biosynthetic process [GO:1905921]; negatively regulated by GO:1905922; positively regulated by positive regulation of acetylcholine biosynthetic process [GO:1905923] Definition: The chemical reactions and pathways resulting in the formation of acetylcholine, the acetic acid ester of the organic base choline. Relationships: is a type of GO:0008291; is a type of GO:0009058